medial membrane band assembly [GO:0032130] (biological process) Definition: The assembly of a sterol-rich region of the plasma membrane at the cell surface overlying the contractile ring. References: PMID:15517003 Also known as: medial membrane band formation Relationships: is_a cellular component assembly [GO:0022607]; is a type of mitotic cytokinetic process [GO:1902410]